{
  "term_label": "negative regulation of epithelial cell proliferation",
  "gene_name": "Cyclin-dependent kinase inhibitor 1B",
  "gene_symbol": "CDKN1B",
  "gene": "UniProtKB:P46527",
  "term_id": "GO:0050680"
}